{
  "term_id": "GO:0005829",
  "gene_name": "Oxysterol-binding protein-related protein 6",
  "gene_symbol": "OSBPL6",
  "gene": "UniProtKB:Q9BZF3",
  "term_label": "cytosol"
}